{
  "term_id": "GO:0007187",
  "gene_name": "Histamine H4 receptor",
  "gene_symbol": "HRH4",
  "term_label": "G protein-coupled receptor signaling pathway, coupled to cyclic nucleotide second messenger",
  "gene": "UniProtKB:Q9H3N8"
}